{
  "gene_name": "Transmembrane emp24 domain-containing protein 10",
  "term_id": "GO:0005793",
  "gene": "UniProtKB:P49755",
  "gene_symbol": "TMED10",
  "term_label": "endoplasmic reticulum-Golgi intermediate compartment"
}